microneme [GO:0020009] (cellular component) Also known as: sarconeme Relationships: is a type of intracellular membrane-bounded organelle [GO:0043231]; is part of GO:0020007 Definition: A small, elongated secretory organelle that forms part of the apical complex, located along the main axis of an apicomplexan parasite cell within the extreme apical region and at the periphery under the inner membrane complex. Of the specialized secretory compartments identified in apicomplexans, micronemes discharge their contents first, during initial contact of the parasite's apical pole with the host cell surface. Micronemal proteins function during parasite attachment and penetration into the target cell. References: PMID:11801218 Sources: ISBN:0521664470